{
  "term_label": "plasma membrane",
  "gene_name": "Vesicle-associated membrane protein 1",
  "gene": "UniProtKB:P23763",
  "term_id": "GO:0005886",
  "gene_symbol": "VAMP1"
}